{
  "gene": "UniProtKB:Q9UGK3",
  "gene_symbol": "STAP2",
  "gene_name": "Signal-transducing adaptor protein 2",
  "term_label": "Unknown molecular function",
  "term_id": "UNKNOWN:0001"
}